{
  "gene": "UniProtKB:Q08828",
  "term_label": "cAMP biosynthetic process",
  "gene_name": "Adenylate cyclase type 1",
  "term_id": "GO:0006171",
  "gene_symbol": "ADCY1"
}